{
  "term_id": "UNKNOWN:0001",
  "gene_name": "Krev interaction trapped protein 1",
  "gene": "UniProtKB:O00522",
  "term_label": "Unknown molecular function",
  "gene_symbol": "KRIT1"
}